negative regulation of urea catabolic process [GO:1901713] (biological process) Definition: Any process that stops, prevents or reduces the frequency, rate or extent of urea catabolic process. Sources: GOC:TermGenie Relationships: is a type of negative regulation of amide catabolic process [GO:0034252]; is a type of GO:0034254; is a type of negative regulation of small molecule metabolic process [GO:0062014]; is a type of negative regulation of nitrogen cycle metabolic process [GO:1903315]; negatively regulates urea catabolic process [GO:0043419] Also known as: down regulation of urea breakdown, down regulation of urea catabolic process, down regulation of urea catabolism, down regulation of urea decomposition, down regulation of urea degradation, down-regulation of urea breakdown, down-regulation of urea catabolic process, down-regulation of urea catabolism, down-regulation of urea decomposition, down-regulation of urea degradation, downregulation of urea breakdown, downregulation of urea catabolic process, downregulation of urea catabolism, downregulation of urea decomposition, downregulation of urea degradation, inhibition of urea breakdown, inhibition of urea catabolism, inhibition of urea decomposition, inhibition of urea degradation, negative regulation of urea breakdown, negative regulation of urea catabolism, negative regulation of urea decomposition, negative regulation of urea degradation, inhibition of urea catabolic process